{
  "gene_name": "Sphingosine kinase 1",
  "gene_symbol": "SPHK1",
  "term_id": "GO:0008481",
  "gene": "UniProtKB:Q9NYA1",
  "term_label": "sphingosine kinase activity"
}